{
  "term_label": "Unknown molecular function",
  "term_id": "UNKNOWN:0001",
  "gene_symbol": "MCEMP1",
  "gene_name": "Mast cell-expressed membrane protein 1",
  "gene": "UniProtKB:Q8IX19"
}